{
  "gene_name": "BPI fold-containing family B member 2",
  "term_label": "Unknown molecular function",
  "gene": "UniProtKB:Q8N4F0",
  "term_id": "UNKNOWN:0001",
  "gene_symbol": "BPIFB2"
}